{
  "gene_symbol": "AQP7",
  "gene": "UniProtKB:O14520",
  "term_id": "GO:0016323",
  "term_label": "basolateral plasma membrane",
  "gene_name": "Aquaporin-7"
}